verbascose biosynthetic process [GO:0033534] (biological process) Sources: GOC:mah Also known as: verbascose anabolism, verbascose biosynthesis, verbascose formation, verbascose synthesis Relationships: is a type of GO:0010325 Definition: The chemical reactions and pathways resulting in the formation of verbascose, the pentasaccharide beta-D-fructofuranosyl alpha-D-galactopyranosyl-(1->6)-alpha-D-galactopyranosyl-(1->6)-alpha-D-galactopyranosyl-(1->6)-alpha-D-glucopyranoside.